{
  "gene_name": "Interleukin-20 receptor subunit beta",
  "term_label": "cytokine receptor activity",
  "term_id": "GO:0004896",
  "gene": "UniProtKB:Q6UXL0",
  "gene_symbol": "IL20RB"
}